{
  "term_label": "low-density lipoprotein particle binding",
  "gene_symbol": "SCARB1",
  "gene_name": "Scavenger receptor class B member 1",
  "gene": "UniProtKB:Q8WTV0",
  "term_id": "GO:0030169"
}